organelle organization [GO:0006996] (biological process) Subtypes: nucleus organization [GO:0006997], mitochondrion organization [GO:0007005], cytoskeleton organization [GO:0007010], endoplasmic reticulum organization [GO:0007029], Golgi organization [GO:0007030], peroxisome organization [GO:0007031], GO:0007033, plastid organization [GO:0009657], vesicle organization [GO:0016050], P granule organization [GO:0030719], GO:0030721, gas vesicle organization [GO:0031412], GO:0034389, rhabdomere development [GO:0042052], bacterial-type flagellum organization [GO:0044781], GO:0044782, GO:0045478, organelle fusion [GO:0048284], GO:0048285, organelle inheritance [GO:0048308], chromosome organization [GO:0051276], GO:0070925, GO:0080119, phagosome maturation [GO:0090382], endoplasmic reticulum-Golgi intermediate compartment organization [GO:0097111], postsynaptic specialization organization [GO:0099084], GO:0106117, glycosome organization [GO:0106233], GO:1903008, subsynaptic reticulum organization [GO:1990255] Note: Note that this term is in the subset of terms that should not be used for direct gene product annotation. Instead, select a child term or, if no appropriate child term exists, please request a new term. Direct annotations to this term may be amended during annotation QC. Sources: GOC:mah Regulation: RO_0002213 by GO:0010638; negatively regulated by GO:0010639; regulated by regulation of organelle organization [GO:0033043] Relationships: is a type of cellular component organization [GO:0016043] Also known as: organelle organisation, single organism organelle organization, organelle organization and biogenesis, single-organism organelle organization Definition: A process that is carried out at the cellular level which results in the assembly, arrangement of constituent parts, or disassembly of an organelle within a cell. An organelle is an organized structure of distinctive morphology and function. Includes the nucleus, mitochondria, plastids, vacuoles, vesicles, ribosomes and the cytoskeleton. Excludes the plasma membrane.